{
  "gene_symbol": "CATSPERZ",
  "gene": "UniProtKB:Q9NTU4",
  "gene_name": "Cation channel sperm-associated auxiliary subunit zeta",
  "term_id": "GO:0030317",
  "term_label": "flagellated sperm motility"
}